{
  "term_id": "UNKNOWN:0003",
  "gene_symbol": "ZDHHC17",
  "gene": "UniProtKB:Q8IUH5",
  "gene_name": "Palmitoyltransferase ZDHHC17",
  "term_label": "Unknown cellular component"
}